{
  "gene_name": "Glycerol kinase",
  "term_id": "GO:0006641",
  "gene_symbol": "GK",
  "gene": "UniProtKB:P32189",
  "term_label": "triglyceride metabolic process"
}